{
  "gene_name": "Checkpoint protein HUS1B",
  "term_id": "UNKNOWN:0001",
  "term_label": "Unknown molecular function",
  "gene_symbol": "HUS1B",
  "gene": "UniProtKB:Q8NHY5"
}